{
  "gene_name": "Unconventional myosin-Ic",
  "gene": "UniProtKB:O00159",
  "term_label": "cytoplasm",
  "term_id": "GO:0005737",
  "gene_symbol": "MYO1C"
}